{
  "gene_name": "Ribose-phosphate pyrophosphokinase 3",
  "gene_symbol": "PRPS1L1",
  "gene": "UniProtKB:P21108",
  "term_id": "GO:0005737",
  "term_label": "cytoplasm"
}